carbon catabolite repression of transcription by galactose [GO:0000410] (biological process) Definition: A transcription regulation process in which the presence of galactose that leads to a decrease in the frequency, rate, or extent of transcription of specific genes involved in the metabolism of other carbon sources. Carbon catabolite repression is a mechanism of genetic regulation which the accumulation of catabolites of one substance in the cell represses the formation of enzymes that contribute to the catabolism of other substances. Sources: GOC:mah Also known as: down regulation of transcription by galactose, down-regulation of transcription by galactose, downregulation of transcription by galactose, inhibition of transcription by galactose Subtypes: carbon catabolite repression of transcription from RNA polymerase II promoter by galactose [GO:0000434] Relationships: is a type of regulation of transcription by galactose [GO:0000409]; is a type of carbon catabolite repression of transcription [GO:0045013]